{
  "term_id": "GO:0034056",
  "gene_name": "Progesterone receptor",
  "gene": "UniProtKB:P06401",
  "term_label": "estrogen response element binding",
  "gene_symbol": "PGR"
}